inositol oxygenase activity [GO:0050113] (molecular function) Also known as: myo-inositol oxygenase activity, MOO activity, meso-inositol oxygenase activity, myo-inositol:oxygen oxidoreductase activity Definition: Catalysis of the reaction: myo-inositol + O2 = D-glucuronate + H2O + H+. Sources: RHEA:23696 Relationships: is a type of monooxygenase activity [GO:0004497]; is a type of GO:0016701